{
  "gene_symbol": "UGT1A8",
  "term_id": "GO:0001889",
  "term_label": "liver development",
  "gene_name": "UDP-glucuronosyltransferase 1A8",
  "gene": "UniProtKB:Q9HAW9"
}